{
  "gene_symbol": "CASP8",
  "term_id": "GO:0005737",
  "term_label": "cytoplasm",
  "gene_name": "Caspase-8",
  "gene": "UniProtKB:Q14790"
}